epithelial cell development [GO:0002064] (biological process) Sources: GOC:dph Definition: The process whose specific outcome is the progression of an epithelial cell over time, from its formation to the mature structure. An epithelial cell is a cell usually found in a two-dimensional sheet with a free surface. Relationships: is a type of cell development [GO:0048468]; is part of epithelial cell differentiation [GO:0030855] Subtypes: endothelial cell development [GO:0001885], columnar/cuboidal epithelial cell development [GO:0002066], pancreatic A cell development [GO:0003322], GO:0003323, pancreatic PP cell development [GO:0003325], keratinocyte development [GO:0003334], follicle cell of egg chamber development [GO:0030707], Sertoli cell development [GO:0060009], granulosa cell development [GO:0060016], GO:0070307, glomerular mesangial cell development [GO:0072144], GO:0072310, glomerular epithelial cell fate commitment [GO:0072314], pancreatic E cell development [GO:0090105]